{
  "term_id": "GO:0007165",
  "gene_symbol": "OR7A2P",
  "term_label": "signal transduction",
  "gene_name": "Putative olfactory receptor 7A2",
  "gene": "UniProtKB:Q8NGA2"
}